{
  "term_label": "antimicrobial humoral immune response mediated by antimicrobial peptide",
  "term_id": "GO:0061844",
  "gene_symbol": "DCD",
  "gene_name": "Dermcidin",
  "gene": "UniProtKB:P81605"
}